regulation of proteasomal ubiquitin-dependent protein catabolic process [GO:0032434] (BP) Subtypes: negative regulation of proteasomal ubiquitin-dependent protein catabolic process [GO:0032435], positive regulation of proteasomal ubiquitin-dependent protein catabolic process [GO:0032436], regulation of SCF-dependent proteasomal ubiquitin-dependent protein catabolic process [GO:0062025], regulation of anaphase-promoting complex-dependent catabolic process [GO:1905784] Definition: Any process that modulates the frequency, rate or extent of the breakdown of a protein or peptide by hydrolysis of its peptide bonds, initiated by the covalent attachment of ubiquitin, and mediated by the proteasome. Sources: GOC:mah Relationships: is a type of regulation of proteasomal protein catabolic process [GO:0061136]; is a type of regulation of ubiquitin-dependent protein catabolic process [GO:2000058]; regulates proteasome-mediated ubiquitin-dependent protein catabolic process [GO:0043161]